{
  "gene_symbol": "WHRN",
  "gene_name": "Whirlin",
  "term_id": "UNKNOWN:0001",
  "term_label": "Unknown molecular function",
  "gene": "UniProtKB:Q9P202"
}